chitin disaccharide deacetylase activity [GO:0036311] (MF) Definition: Catalysis of the reaction: H2O + N,N'-diacetylchitobiose = acetate + N-acetyl-beta-D-glucosaminyl-(1->4)-D-glucosamine. Sources: RHEA:27469 Also known as: chitin oligosaccharide amidohydrolase activity, chitin oligosaccharide deacetylase activity, chitobiose amidohydrolase activity Note: In contrast to EC:3.5.1.41 (chitin deacetylase) this enzyme is specific for the chitin disaccharide. Relationships: is a type of hydrolase activity, acting on carbon-nitrogen (but not peptide) bonds, in linear amides [GO:0016811]